{
  "gene": "UniProtKB:Q6PF05",
  "term_id": "UNKNOWN:0002",
  "gene_symbol": "TTC23L",
  "term_label": "Unknown biological process",
  "gene_name": "Tetratricopeptide repeat protein 23-like"
}